{
  "gene_symbol": "ZFHX4",
  "gene": "UniProtKB:Q86UP3",
  "term_label": "DNA-binding transcription factor activity, RNA polymerase II-specific",
  "term_id": "GO:0000981",
  "gene_name": "Zinc finger homeobox protein 4"
}